{
  "gene_name": "Putative small nuclear ribonucleoprotein G-like protein 15",
  "gene": "UniProtKB:A8MWD9",
  "term_label": "U1 snRNP",
  "gene_symbol": "SNRPGP15",
  "term_id": "GO:0005685"
}